{
  "term_label": "cell migration",
  "gene_symbol": "PIK3CD",
  "gene": "UniProtKB:O00329",
  "gene_name": "Phosphatidylinositol 4,5-bisphosphate 3-kinase catalytic subunit delta isoform",
  "term_id": "GO:0016477"
}